{
  "term_id": "GO:0009083",
  "gene_name": "2-oxoisovalerate dehydrogenase subunit beta, mitochondrial",
  "term_label": "branched-chain amino acid catabolic process",
  "gene_symbol": "BCKDHB",
  "gene": "UniProtKB:P21953"
}